{
  "gene": "UniProtKB:Q8IV13",
  "gene_symbol": "CCNJL",
  "term_label": "nucleus",
  "gene_name": "Cyclin-J-like protein",
  "term_id": "GO:0005634"
}